{
  "gene_symbol": "LYPD5",
  "term_label": "Unknown biological process",
  "term_id": "UNKNOWN:0002",
  "gene": "UniProtKB:Q6UWN5",
  "gene_name": "Ly6_PLAUR domain-containing protein 5"
}